{
  "gene": "UniProtKB:Q9GZV1",
  "gene_name": "Ankyrin repeat domain-containing protein 2",
  "gene_symbol": "ANKRD2",
  "term_label": "nucleus",
  "term_id": "GO:0005634"
}